{
  "gene_name": "Ceramide kinase-like protein",
  "term_label": "lipid kinase activity",
  "gene_symbol": "CERKL",
  "term_id": "GO:0001727",
  "gene": "UniProtKB:Q49MI3"
}